patched ligand maturation [GO:0007225] (biological process) Relationships: is a type of peptide hormone processing [GO:0016486] Also known as: hh protein processing, Hedgehog protein processing, patched ligand processing References: PMID:15057936 Definition: The posttranslational modification of members of the Hedgehog family of signaling proteins in order for Hedgehog to exert its biological activity. These modifications include cleavage of its signal sequence, autocatalytic protein cleavage and the attachment of sterol groups.